{
  "gene_symbol": "ZMIZ2",
  "term_id": "GO:0006357",
  "gene": "UniProtKB:Q8NF64",
  "term_label": "regulation of transcription by RNA polymerase II",
  "gene_name": "Zinc finger MIZ domain-containing protein 2"
}